o-pyrocatechuate decarboxylase activity [GO:0050150] (molecular function) Definition: Catalysis of the reaction: 2,3-dihydroxybenzoate + H+ = catechol + CO2. Sources: EC:4.1.1.46, RHEA:21492 Also known as: 2,3-dihydroxybenzoate decarboxylase activity, 2,3-DHBA decarboxylase activity, 2,3-dihydroxybenzoate carboxy-lyase (catechol-forming), 2,3-dihydroxybenzoate carboxy-lyase activity, 2,3-dihydroxybenzoic acid decarboxylase activity Relationships: is a type of carboxy-lyase activity [GO:0016831]